{
  "term_label": "Unknown biological process",
  "term_id": "UNKNOWN:0002",
  "gene": "UniProtKB:Q8NFZ4",
  "gene_symbol": "NLGN2",
  "gene_name": "Neuroligin-2"
}